{
  "gene_symbol": "INSR",
  "term_id": "GO:0043410",
  "term_label": "positive regulation of MAPK cascade",
  "gene_name": "Insulin receptor",
  "gene": "UniProtKB:P06213"
}